2,2-dialkylglycine decarboxylase (pyruvate) activity [GO:0047432] (molecular function) Definition: Catalysis of the reaction: 2,2-dialkylglycine + H+ + pyruvate = L-alanine + CO2 + dialkyl ketone. Relationships: is a type of carboxy-lyase activity [GO:0016831] Sources: EC:4.1.1.64, RHEA:16073 Also known as: 2,2-dialkyl-2-amino acid-pyruvate aminotransferase activity, 2,2-dialkylglycine carboxy-lyase (amino-transferring), 2,2-dialkylglycine carboxy-lyase (amino-transferring; L-alanine-forming), L-alanine-alpha-ketobutyrate aminotransferase activity, alpha-dialkyl amino acid transaminase activity, dialkyl amino acid (pyruvate) decarboxylase activity, dialkylamino-acid decarboxylase (pyruvate)